positive regulation of protein export from nucleus [GO:0046827] (biological process) Sources: GOC:bf Relationships: is_a positive regulation of nucleocytoplasmic transport [GO:0046824]; is a type of regulation of protein export from nucleus [GO:0046825]; is a type of positive regulation of intracellular protein transport [GO:0090316]; positively regulates GO:0006611 Definition: Any process that activates or increases the frequency, rate or extent of directed movement of proteins from the nucleus into the cytoplasm. Also known as: positive regulation of protein export from cell nucleus, positive regulation of protein export out of nucleus, positive regulation of protein transport from nucleus to cytoplasm, positive regulation of protein-nucleus export, up regulation of protein export from nucleus, up-regulation of protein export from nucleus, upregulation of protein export from nucleus, activation of protein export from nucleus, stimulation of protein export from nucleus Subtypes: positive regulation of protein export from nucleus in response to glucose starvation [GO:0036279], GO:1900199